{
  "term_label": "protein ubiquitination",
  "term_id": "GO:0016567",
  "gene_name": "RING finger protein 44",
  "gene_symbol": "RNF44",
  "gene": "UniProtKB:Q7L0R7"
}